{
  "gene_name": "Beta-1,3-N-acetylglucosaminyltransferase lunatic fringe",
  "gene_symbol": "LFNG",
  "gene": "UniProtKB:Q8NES3",
  "term_label": "O-fucosylpeptide 3-beta-N-acetylglucosaminyltransferase activity",
  "term_id": "GO:0033829"
}